{
  "gene_symbol": "SLC34A1",
  "gene": "UniProtKB:Q06495",
  "term_id": "GO:0030643",
  "gene_name": "Sodium-dependent phosphate transport protein 2A",
  "term_label": "intracellular phosphate ion homeostasis"
}